{
  "gene_name": "Transducin-like enhancer protein 4",
  "gene": "UniProtKB:Q04727",
  "term_id": "GO:0005667",
  "term_label": "transcription regulator complex",
  "gene_symbol": "TLE4"
}